3,4-dihydroxy-9,10-secoandrosta-1,3,5(10)-triene-9,17-dione 4,5-dioxygenase activity [GO:0047071] (molecular function) Definition: Catalysis of the reaction: 3,4-dihydroxy-9,10-secoandrosta-1,3,5(10)-triene-9,17-dione + O2 = 3-hydroxy-5,9,17-trioxo-4,5:9,10-disecoandrosta-1(10),2-dien-4-oate + H+. Also known as: steroid 4,5-dioxygenase activity, 3,4-dihydroxy-9,10-secoandrosta-1,3,5(10)-triene-9,17-dione:oxygen 4,5-oxidoreductase (decyclizing), 3-alkylcatechol 2,3-dioxygenase activity Relationships: is a type of oxidoreductase activity, acting on single donors with incorporation of molecular oxygen, incorporation of two atoms of oxygen [GO:0016702] Sources: EC:1.13.11.25, RHEA:21352